{
  "term_id": "GO:0030169",
  "gene_symbol": "CRP",
  "term_label": "low-density lipoprotein particle binding",
  "gene_name": "C-reactive protein",
  "gene": "UniProtKB:P02741"
}